{
  "term_label": "plasma membrane",
  "gene_symbol": "TMEM204",
  "gene": "UniProtKB:Q9BSN7",
  "gene_name": "Transmembrane protein 204",
  "term_id": "GO:0005886"
}